{
  "term_id": "GO:0019814",
  "gene": "UniProtKB:P01721",
  "gene_name": "Immunoglobulin lambda variable 6-57",
  "term_label": "immunoglobulin complex",
  "gene_symbol": "IGLV6-57"
}